{
  "gene": "UniProtKB:Q7L0R7",
  "term_id": "UNKNOWN:0003",
  "gene_name": "RING finger protein 44",
  "gene_symbol": "RNF44",
  "term_label": "Unknown cellular component"
}